glycerate transmembrane transporter activity [GO:1901974] (molecular function) Relationships: is a type of monocarboxylic acid transmembrane transporter activity [GO:0008028]; is a type of GO:0015144; is_a GO:0042879; is part of GO:1901975 References: PMID:23382251 Sources: GOC:TermGenie Definition: Enables the transfer of glycerate from one side of a membrane to the other.